{
  "gene_symbol": "NARS1",
  "term_id": "GO:0005737",
  "gene": "UniProtKB:O43776",
  "term_label": "cytoplasm",
  "gene_name": "Asparagine--tRNA ligase, cytoplasmic"
}